dorsal/ventral pattern formation, imaginal disc [GO:0007450] (biological process) Relationships: is a type of imaginal disc pattern formation [GO:0007447]; is a type of dorsal/ventral pattern formation [GO:0009953] Definition: The establishment, maintenance and elaboration of the dorsal/ventral axis of the imaginal disc. Imaginal disks are masses of hypodermic cells, carried by the larvae of some insects after leaving the egg, from which masses the wings and legs of the adult are subsequently formed. Subtypes: GO:0048190 Also known as: dorsal-ventral pattern formation, imaginal disc, dorsoventral pattern formation, imaginal disc Sources: GOC:jid, ISBN:0879694238